terminal cell fate specification, open tracheal system [GO:0035154] (biological process) Definition: The process in which a cell in an open tracheal system becomes capable of differentiating autonomously into a terminal cell in an environment that is neutral with respect to the developmental pathway; upon specification, the cell fate can be reversed. Terminal cells send long and bifurcated hollow branches toward target tissues to allow oxygen exchange. Relationships: is a type of epithelial cell type specification, open tracheal system [GO:0035153] References: PMID:10684581, PMID:11063940 Sources: GOC:mtg_sensu Also known as: terminal cell fate specification Regulation: RO_0002212 by GO:0035155